cholesterol-protein transferase activity [GO:0140853] (molecular function) Definition: Catalysis of the reaction: cholesterol + glycyl-L-cysteinyl-[protein] + H+ = [protein]-C-terminal glycyl cholesterol ester + N-terminal L-cysteinyl-[protein]. Relationships: is a type of GO:0016740; is a type of GO:0140096 References: PMID:8824192 Sources: RHEA:59504 Also known as: cholesterol transferase activity